{
  "term_label": "protein kinase binding",
  "gene_symbol": "LRRC7",
  "gene": "UniProtKB:Q96NW7",
  "term_id": "GO:0019901",
  "gene_name": "Leucine-rich repeat-containing protein 7"
}